{
  "gene_symbol": "TRGV11",
  "gene": "UniProtKB:A0A075B6L2",
  "term_id": "UNKNOWN:0001",
  "gene_name": "Probable non-functional T cell receptor gamma variable 11",
  "term_label": "Unknown molecular function"
}